mesonephric nephron epithelium development [GO:0061241] (biological process) Subtypes: mesonephric macula densa development [GO:0061220], GO:0061232, GO:0061242 Definition: The process whose specific outcome is the progression of the mesonephric nephron epithelium over time, from its formation to the mature structure. An epithelium is a tissue that covers the internal or external surfaces of an anatomical structure. The mesonephric nephron epithelium is a tissue that covers the surface of a nephron in the mesonephros. Relationships: is a type of nephron epithelium development [GO:0072009]; is a type of GO:0072163; is part of mesonephric nephron development [GO:0061215] Sources: GOC:mtg_kidney_jan10